{
  "term_label": "endosomal transport",
  "gene": "UniProtKB:Q9H0R1",
  "gene_symbol": "AP5M1",
  "term_id": "GO:0016197",
  "gene_name": "AP-5 complex subunit mu-1"
}